{
  "gene_name": "Putative uncharacterized protein PIK3CD-AS1",
  "gene": "UniProtKB:Q5SR53",
  "gene_symbol": "PIK3CD-AS1",
  "term_label": "Unknown cellular component",
  "term_id": "UNKNOWN:0003"
}